{
  "term_label": "Unknown biological process",
  "gene": "UniProtKB:Q9P0M2",
  "gene_symbol": "AKAP7",
  "gene_name": "A-kinase anchor protein 7 isoform gamma",
  "term_id": "UNKNOWN:0002"
}